{
  "gene_name": "Alkaline ceramidase 3",
  "term_label": "endoplasmic reticulum membrane",
  "gene": "UniProtKB:Q9NUN7",
  "term_id": "GO:0005789",
  "gene_symbol": "ACER3"
}